{
  "gene": "UniProtKB:P0C7W6",
  "term_label": "Unknown biological process",
  "gene_symbol": "CCDC172",
  "term_id": "UNKNOWN:0002",
  "gene_name": "Coiled-coil domain-containing protein 172"
}